pyrimidine nucleoside transmembrane transporter activity [GO:0015214] (molecular function) Definition: Enables the transfer of a pyrimidine nucleoside, a pyrimidine base covalently bonded to a ribose or deoxyribose sugar from one side of a membrane to the other. Sources: GOC:ai Relationships: is a type of nucleoside transmembrane transporter activity [GO:0005337]; is part of pyrimidine-containing compound transmembrane transport [GO:0072531] Subtypes: cytidine transmembrane transporter activity [GO:0015212], GO:0015213